{
  "term_label": "chromatin",
  "gene_symbol": "JMJD1C",
  "gene_name": "Probable JmjC domain-containing histone demethylation protein 2C",
  "gene": "UniProtKB:Q15652",
  "term_id": "GO:0000785"
}